{
  "term_id": "GO:0006357",
  "gene_symbol": "ZNF470",
  "gene_name": "Zinc finger protein 470",
  "term_label": "regulation of transcription by RNA polymerase II",
  "gene": "UniProtKB:Q6ECI4"
}